{
  "term_label": "9+0 non-motile cilium",
  "gene_symbol": "IFTAP",
  "term_id": "GO:0097731",
  "gene": "UniProtKB:Q86VG3",
  "gene_name": "Intraflagellar transport-associated protein"
}